{
  "gene_symbol": "TRIM23",
  "term_id": "GO:0016192",
  "term_label": "vesicle-mediated transport",
  "gene_name": "E3 ubiquitin-protein ligase TRIM23",
  "gene": "UniProtKB:P36406"
}